{
  "gene_name": "Protein C-ets-2",
  "gene": "UniProtKB:P15036",
  "term_id": "GO:0030154",
  "gene_symbol": "ETS2",
  "term_label": "cell differentiation"
}